{
  "gene": "UniProtKB:Q9UBP6",
  "term_label": "RNA (guanine-N7)-methylation",
  "gene_symbol": "METTL1",
  "gene_name": "tRNA (guanine-N(7)-)-methyltransferase",
  "term_id": "GO:0036265"
}